{
  "term_label": "base-excision repair",
  "gene_name": "DNA polymerase beta",
  "term_id": "GO:0006284",
  "gene": "UniProtKB:P06746",
  "gene_symbol": "POLB"
}